{
  "gene": "UniProtKB:Q9H4B8",
  "gene_symbol": "DPEP3",
  "term_label": "Unknown molecular function",
  "gene_name": "Dipeptidase 3",
  "term_id": "UNKNOWN:0001"
}